S-(hydroxymethyl)glutathione dehydrogenase [NAD(P)+] activity [GO:0051903] (molecular function) Definition: Catalysis of the reaction: S-(hydroxymethyl)glutathione + NAD(P)+ = S-formylglutathione + NAD(P)H + H+. Sources: EC:1.1.1.284 Also known as: ADH3 activity, chi-ADH activity, FDH activity, GD-FALDH activity, GS-FDH activity, NAD- and glutathione-dependent formaldehyde dehydrogenase activity, NAD-dependent formaldehyde dehydrogenase activity, NAD-linked formaldehyde dehydrogenase activity, S-(hydroxymethyl)glutathione:NAD+ oxidoreductase activity, class III alcohol dehydrogenase activity, formic dehydrogenase activity, glutathione-dependent formaldehyde dehydrogenase activity Relationships: is a type of GO:0016616 Subtypes: S-(hydroxymethyl)glutathione dehydrogenase (NADP+) activity [GO:0106321], S-(hydroxymethyl)glutathione dehydrogenase (NAD+) activity [GO:0106322]